{
  "gene": "UniProtKB:Q9H4M9",
  "gene_name": "EH domain-containing protein 1",
  "gene_symbol": "EHD1",
  "term_id": "GO:0072659",
  "term_label": "protein localization to plasma membrane"
}